{
  "gene_symbol": "NANOG",
  "term_label": "nucleus",
  "gene": "UniProtKB:Q9H9S0",
  "gene_name": "Homeobox protein NANOG",
  "term_id": "GO:0005634"
}